{
  "term_id": "GO:0009435",
  "term_label": "NAD+ biosynthetic process",
  "gene_name": "Nicotinamide phosphoribosyltransferase",
  "gene": "UniProtKB:P43490",
  "gene_symbol": "NAMPT"
}